{
  "gene": "UniProtKB:Q9Y296",
  "gene_name": "Trafficking protein particle complex subunit 4",
  "term_id": "GO:0006888",
  "gene_symbol": "TRAPPC4",
  "term_label": "endoplasmic reticulum to Golgi vesicle-mediated transport"
}